{
  "gene_symbol": "IGKJ2",
  "term_id": "UNKNOWN:0002",
  "gene": "UniProtKB:A0A0A0MT85",
  "gene_name": "Immunoglobulin kappa joining 2 (Fragment)",
  "term_label": "Unknown biological process"
}